mating projection membrane [GO:0070250] (cellular component) Sources: GOC:jp Relationships: is a type of GO:0031253; BFO_0000050 mating projection [GO:0005937] Definition: The portion of the plasma membrane surrounding a mating projection, the projection formed by unicellular fungi in response to mating pheromone. Also known as: shmoo membrane